mercury ion binding [GO:0045340] (molecular function) Relationships: is a type of GO:0046914 Definition: Binding to a mercury ion (Hg2+). Also known as: Hg ion binding, mercury binding Sources: GOC:go_curators